transmembrane receptor protein tyrosine phosphatase activity [GO:0005001] (molecular function) References: PMID:34353440 Relationships: is a type of protein tyrosine phosphatase activity [GO:0004725]; is a type of GO:0019198 Definition: Combining with a signal and transmitting the signal from one side of the membrane to the other to initiate a change in cell activity by catalysis of the reaction: protein tyrosine phosphate + H2O = protein tyrosine + phosphate.